{
  "term_id": "GO:0004252",
  "gene_symbol": "FURIN",
  "gene_name": "Furin",
  "gene": "UniProtKB:P09958",
  "term_label": "serine-type endopeptidase activity"
}